DNA N-glycosylase activity [GO:0019104] (molecular function) Subtypes: mismatch base pair DNA N-glycosylase activity [GO:0000700], oxidized base lesion DNA N-glycosylase activity [GO:0000702], pyrimidine dimer DNA N-glycosylase activity [GO:0000704], alkylbase DNA N-glycosylase activity [GO:0003905], GO:0097506 Also known as: DNA glycosylase activity, endonuclease VIII activity Definition: Catalysis of the removal of damaged bases by cleaving the N-C1' glycosidic bond between the target damaged DNA base and the deoxyribose sugar. The reaction releases a free base and leaves an apurinic/apyrimidinic (AP) site. References: PMID:11554296 Sources: GOC:elh Relationships: is a type of GO:0016799; is a type of catalytic activity, acting on DNA [GO:0140097]